{
  "gene": "UniProtKB:P11233",
  "term_id": "GO:0017157",
  "term_label": "regulation of exocytosis",
  "gene_name": "Ras-related protein Ral-A",
  "gene_symbol": "RALA"
}